{
  "term_label": "Unknown biological process",
  "term_id": "UNKNOWN:0002",
  "gene_name": "Bridge-like lipid transfer protein family member 3B",
  "gene_symbol": "BLTP3B",
  "gene": "UniProtKB:A0JNW5"
}